{
  "gene": "UniProtKB:P36897",
  "gene_symbol": "TGFBR1",
  "term_label": "heart development",
  "gene_name": "TGF-beta receptor type-1",
  "term_id": "GO:0007507"
}